hyphal tip polarisome [GO:0031562] (cellular component) Relationships: is a type of polarisome [GO:0000133]; is part of GO:0001411 Definition: Protein complex that has a role in determining cell polarity, found at the tip of a growing fungal hypha. References: PMID:15976451